{
  "gene_symbol": "PLA2G4A",
  "gene": "UniProtKB:P47712",
  "gene_name": "Cytosolic phospholipase A2",
  "term_id": "GO:0046475",
  "term_label": "glycerophospholipid catabolic process"
}